{
  "gene": "UniProtKB:Q12788",
  "gene_name": "Transducin beta-like protein 3",
  "gene_symbol": "TBL3",
  "term_id": "GO:0034511",
  "term_label": "U3 snoRNA binding"
}